methylamine metabolic process [GO:0030416] (biological process) Definition: The chemical reactions and pathways involving methylamine (CH3NH2). Sources: ISBN:0721662544 Relationships: is a type of amine metabolic process [GO:0009308] Also known as: methylamine metabolism, methylammonium metabolic process, methylammonium metabolism Subtypes: methane biosynthetic process from methylamine [GO:2001128]